{
  "gene_name": "DNA-directed RNA polymerase III subunit RPC2",
  "gene_symbol": "POLR3B",
  "term_label": "RNA polymerase III complex",
  "gene": "UniProtKB:Q9NW08",
  "term_id": "GO:0005666"
}